epidermis morphogenesis involved in nipple formation [GO:0060660] (biological process) Relationships: is a type of epidermis morphogenesis [GO:0048730]; is part of nipple morphogenesis [GO:0060658] References: PMID:12558599 Sources: GOC:dph Definition: The process in which the epidermis of the nipple sheath is uplifted to form an umbrella-like projection.